{
  "term_label": "cysteine-tRNA ligase activity",
  "gene_name": "Cysteine--tRNA ligase, cytoplasmic",
  "gene_symbol": "CARS1",
  "term_id": "GO:0004817",
  "gene": "UniProtKB:P49589"
}